glomerular basement membrane development [GO:0032836] (biological process) Definition: The process whose specific outcome is the progression of the glomerular basement membrane over time, from its formation to the mature structure. The glomerular basement membrane is the basal laminal portion of the glomerulus which performs the actual filtration. Sources: GOC:sr Relationships: is a type of GO:0030198; is a type of anatomical structure development [GO:0048856]; is part of glomerulus development [GO:0032835] Subtypes: mesonephric glomerular basement membrane development [GO:0061233], GO:0072274